{
  "gene": "UniProtKB:P23415",
  "gene_name": "Glycine receptor subunit alpha-1",
  "term_label": "excitatory extracellular ligand-gated monoatomic ion channel activity",
  "gene_symbol": "GLRA1",
  "term_id": "GO:0005231"
}